{
  "gene_symbol": "RNF10",
  "gene": "UniProtKB:Q8N5U6",
  "term_id": "GO:1990116",
  "term_label": "ribosome-associated ubiquitin-dependent protein catabolic process",
  "gene_name": "E3 ubiquitin-protein ligase RNF10"
}